protein deadenylylation [GO:0044602] (biological process) Definition: The removal of an adenylyl group (adenosine 5'-monophosphate; AMP) from a protein amino acid. Relationships: is a type of protein denucleotidylation [GO:0044601] Also known as: protein deAMPylation References: PMID:21734656 Sources: GOC:sp